{
  "gene_symbol": "Q1RN00",
  "term_label": "Unknown molecular function",
  "gene_name": "Putative uncharacterized protein LOC151760",
  "gene": "UniProtKB:Q1RN00",
  "term_id": "UNKNOWN:0001"
}